regulation of pseudohyphal growth [GO:2000220] (biological process) Sources: GOC:mah Relationships: is_a GO:0001558; is_a GO:0070784; regulates pseudohyphal growth [GO:0007124] Definition: Any process that modulates the frequency, rate or extent of pseudohyphal growth. Subtypes: negative regulation of pseudohyphal growth [GO:2000221], GO:2000222